{
  "gene_symbol": "SULT1B1",
  "gene_name": "Sulfotransferase 1B1",
  "term_id": "GO:0051923",
  "gene": "UniProtKB:O43704",
  "term_label": "sulfation"
}